{
  "gene": "UniProtKB:Q9BQJ4",
  "gene_symbol": "TMEM47",
  "gene_name": "Transmembrane protein 47",
  "term_id": "UNKNOWN:0001",
  "term_label": "Unknown molecular function"
}